{
  "term_label": "Unknown cellular component",
  "gene": "UniProtKB:Q9NVD3",
  "gene_name": "SET domain-containing protein 4",
  "gene_symbol": "SETD4",
  "term_id": "UNKNOWN:0003"
}